negative regulation of respiratory gaseous exchange [GO:1903941] (biological process) Definition: Any process that stops, prevents or reduces the frequency, rate or extent of respiratory gaseous exchange. Also known as: down regulation of respiratory gaseous exchange, down-regulation of respiratory gaseous exchange, downregulation of respiratory gaseous exchange, inhibition of respiratory gaseous exchange References: PMID:22819705 Sources: GOC:TermGenie, GO_REF:0000058 Relationships: is a type of regulation of respiratory gaseous exchange [GO:0043576]; is a type of GO:0051241; RO_0002212 respiratory gaseous exchange by respiratory system [GO:0007585]